D-alanine catabolic process [GO:0055130] (BP) Definition: The chemical reactions and pathways resulting in the breakdown of D-alanine, the D-enantiomer of the amino acid alanine. Sources: GOC:ecd Relationships: is a type of GO:0006524; is a type of D-amino acid catabolic process [GO:0019478]; is a type of D-alanine metabolic process [GO:0046436] Also known as: (2R)-2-aminopropanoic acid catabolic process